formimidoylglutamase activity [GO:0050415] (molecular function) Relationships: is_a hydrolase activity, acting on carbon-nitrogen (but not peptide) bonds, in linear amidines [GO:0016813] Definition: Catalysis of the reaction: N-formimidoyl-L-glutamate + H2O = L-glutamate + formamide. Sources: EC:3.5.3.8, RHEA:22492 Also known as: formiminoglutamase activity, N-formimidoyl-L-glutamate formimidoylhydrolase activity, N-formimino-L-glutamate formiminohydrolase activity, N-formiminoglutamate hydrolase activity, formiminoglutamate hydrolase activity